{
  "term_label": "cellular response to interleukin-6",
  "gene_symbol": "SBNO2",
  "term_id": "GO:0071354",
  "gene_name": "Protein strawberry notch homolog 2",
  "gene": "UniProtKB:Q9Y2G9"
}